{
  "term_id": "UNKNOWN:0003",
  "gene_name": "Small integral membrane protein 27",
  "gene_symbol": "SMIM27",
  "term_label": "Unknown cellular component",
  "gene": "UniProtKB:A0A1B0GUW7"
}